{
  "gene_name": "Lysozyme C",
  "gene": "UniProtKB:P61626",
  "term_id": "GO:0050830",
  "gene_symbol": "LYZ",
  "term_label": "defense response to Gram-positive bacterium"
}